{
  "term_label": "extracellular space",
  "gene_symbol": "LIPI",
  "term_id": "GO:0005615",
  "gene_name": "Lipase member I",
  "gene": "UniProtKB:Q6XZB0"
}